posterior lateral line ganglion neuron differentiation [GO:0048928] (BP) Definition: The process in which a relatively unspecialized cell acquires specialized features of a neuron of the posterior lateral line ganglion. References: PMID:15018940 Relationships: is a type of lateral line ganglion neuron differentiation [GO:0048891]; BFO_0000050 posterior lateral line ganglion development [GO:0048917]